foam cell differentiation [GO:0090077] (biological process) Subtypes: macrophage derived foam cell differentiation [GO:0010742], smooth muscle derived foam cell differentiation [GO:0090078] Definition: The process in which a relatively unspecialized cell acquires the specialized features of a foam cell. A foam cell is a type of cell containing lipids in small vacuoles and typically seen in atherosclerotic lesions, as well as other conditions. Relationships: is a type of cell differentiation [GO:0030154] Sources: GOC:BHF, GOC:add, GOC:dph, GOC:tb